{
  "term_id": "GO:0019843",
  "gene_name": "Small ribosomal subunit protein uS7",
  "gene": "UniProtKB:P46782",
  "gene_symbol": "RPS5",
  "term_label": "rRNA binding"
}